{
  "gene_symbol": "AKR1D1",
  "gene": "UniProtKB:P51857",
  "term_id": "GO:0008209",
  "term_label": "androgen metabolic process",
  "gene_name": "Aldo-keto reductase family 1 member D1"
}